poly-hydroxybutyrate biosynthetic process [GO:0042619] (biological process) References: PMID:18640095 Sources: GOC:jl Also known as: PHB biosynthesis, PHB biosynthetic process, poly-hydroxybutyrate anabolism, poly-hydroxybutyrate biosynthesis, poly-hydroxybutyrate formation, poly-hydroxybutyrate synthesis Definition: The chemical reactions and pathways resulting in the formation of poly-hydroxybutyrate (PHB), a polymer of beta-hydroxybutyrate and a common storage material of prokaryotic cells. Relationships: is a type of poly-hydroxybutyrate metabolic process [GO:0042618]; is a type of poly(hydroxyalkanoate) biosynthetic process [GO:1901441]